aggressive behavior [GO:0002118] (biological process) Definition: A behavioral interaction between organisms in which one organism has the intention of inflicting physical damage on another individual. Relationships: is a type of behavior [GO:0007610] Subtypes: GO:0002121, fear-induced aggressive behavior [GO:0002122], irritable aggressive behavior [GO:0002123], GO:0002124, maternal aggressive behavior [GO:0002125], instrumental aggressive behavior [GO:0002126] Sources: GOC:hjd Also known as: aggression